regulation of retrograde trans-synaptic signaling by trans-synaptic protein complex [GO:0099176] (biological process) Definition: Any process that modulates the frequency, rate or extent of retrograde trans-synaptic signaling by a trans-synaptic complex. References: PMID:23209303 Sources: GOC:dos Also known as: regulation of trans-synaptic complex mediated retrograde trans-synaptic signaling Relationships: is a type of GO:0099177; regulates retrograde trans-synaptic signaling by trans-synaptic protein complex [GO:0098942]